{
  "term_id": "GO:0098574",
  "gene_name": "LITAF domain-containing protein",
  "gene_symbol": "LITAFD",
  "gene": "UniProtKB:A0A1B0GVX0",
  "term_label": "cytoplasmic side of lysosomal membrane"
}